{
  "gene_symbol": "HEY2",
  "term_label": "anterior/posterior pattern specification",
  "gene_name": "Hairy_enhancer-of-split related with YRPW motif protein 2",
  "gene": "UniProtKB:Q9UBP5",
  "term_id": "GO:0009952"
}